{
  "gene_name": "Transmembrane 4 L6 family member 18",
  "gene_symbol": "TM4SF18",
  "term_id": "UNKNOWN:0002",
  "term_label": "Unknown biological process",
  "gene": "UniProtKB:Q96CE8"
}